adult feeding behavior [GO:0008343] (biological process) Definition: Feeding behavior in a fully developed and mature organism. Relationships: is a type of GO:0007631; is a type of adult behavior [GO:0030534] Also known as: adult feeding behaviour Note: See also the biological process term 'feeding behavior ; GO:0007631'. Sources: GOC:mah